myeloid progenitor cell differentiation [GO:0002318] (biological process) Regulation: regulated by regulation of myeloid progenitor cell differentiation [GO:1905453]; negatively regulated by GO:1905454; positively regulated by positive regulation of myeloid progenitor cell differentiation [GO:1905455] References: PMID:16551264 Sources: GOC:add Relationships: is a type of GO:0002244 Definition: The process in which a precursor cell type acquires the specialized features of a myeloid progenitor cell. Myeloid progenitor cells include progenitor cells for any of the myeloid lineages.